deoxyguanosine biosynthetic process [GO:0042452] (biological process) Definition: The chemical reactions and pathways resulting in the formation of deoxyguanosine, a nucleoside consisting of the base guanine and the sugar deoxyribose. Sources: GOC:jl Also known as: deoxyguanosine anabolism, deoxyguanosine biosynthesis, deoxyguanosine formation, deoxyguanosine synthesis Relationships: is a type of purine deoxyribonucleoside biosynthetic process [GO:0046123] Subtypes: deoxyguanosine salvage [GO:0006180]